{
  "gene": "UniProtKB:Q6UX04",
  "term_id": "UNKNOWN:0002",
  "gene_name": "Spliceosome-associated protein CWC27 homolog",
  "gene_symbol": "CWC27",
  "term_label": "Unknown biological process"
}